{
  "gene": "UniProtKB:P05549",
  "term_id": "GO:0001822",
  "gene_symbol": "TFAP2A",
  "term_label": "kidney development",
  "gene_name": "Transcription factor AP-2-alpha"
}